{
  "term_label": "plasma membrane",
  "gene_symbol": "OR2J1",
  "term_id": "GO:0005886",
  "gene": "UniProtKB:Q9GZK6",
  "gene_name": "Olfactory receptor 2J1"
}